{
  "gene": "UniProtKB:A0A075B734",
  "term_id": "GO:0015793",
  "gene_symbol": "AQP7B",
  "term_label": "glycerol transmembrane transport",
  "gene_name": "Aquaporin-7B"
}